histone H3K27me3 reader activity [GO:0061628] (molecular function) Note: Comment: Note that the residue position corresponds to the canonical human H3 histone (UniProtKB:P84243); this residue is conserved across all eukaryotes. Residue 1 is the first residue following removal of the initiating Methionine (Met). Note that each histone is encoded by multiple genes, and sequences may vary across different genes within an organism. Relationships: is a type of histone H3 reader activity [GO:0140006] References: PMID:23948251 Sources: GOC:dph Definition: A histone reader that recognizes a histone H3 trimethylated at lysine 27. Also known as: H3K27me3 modified histone binding, histone H3-K27me3 modified histone binding